{
  "gene_name": "Coiled-coil domain-containing protein 201",
  "gene_symbol": "CCDC201",
  "gene": "UniProtKB:A0A1B0GTI1",
  "term_label": "Unknown molecular function",
  "term_id": "UNKNOWN:0001"
}